sodium:bicarbonate symporter activity [GO:0008510] (molecular function) Relationships: is a type of solute:sodium symporter activity [GO:0015370]; is a type of monoatomic cation:bicarbonate symporter activity [GO:0140410] Also known as: sodium/bicarbonate cotransporter activity, sodium:bicarbonate cotransporter activity, sodium:hydrogencarbonate symporter activity Definition: Enables the transfer of a solute or solutes from one side of a membrane to the other according to the reaction: Na+(out) + HCO3-(out) = Na+(in) + HCO3-(in). Sources: TC:2.A.31.2.1